TIM22 mitochondrial import inner membrane insertion complex [GO:0042721] (cellular component) Definition: A multi-subunit complex embedded in the mitochondrial inner membrane that mediates the inner membrane insertion of multi-transmembrane spanning proteins that contain internal targeting elements. In yeast cells, TIM22 is a 300-kDa complex, consisting of four membrane integral subunits, Tim22, Tim54, Tim18 and Sdh3, and a peripheral chaperone complex consisting of the small TIM proteins, Tim9-Tim10-Tim12. References: PMID:12191765, PMID:27554484 Relationships: is a type of inner mitochondrial membrane protein complex [GO:0098800] Also known as: mitochondrial protein translocase complex, Tim22 complex, mitochondrial inner membrane protein insertion complex